neural crest-derived cardiac fibroblast cell differentiation [GO:0060942] (biological process) Sources: GOC:mtg_heart Definition: The process in which a neural crest cell acquires the specialized structural and/or functional features of a cardiac fibroblast. A cardiac fibroblast is a connective tissue cell in the heart which secretes an extracellular matrix rich in collagen and other macromolecules. Relationships: is a type of cardiac fibroblast cell differentiation [GO:0060935]